phagosome reneutralization [GO:0044655] (biological process) Definition: Any process that increases the pH of the phagosome, measured by the concentration of the hydrogen ion, as part of the process of phagosome maturation. Relationships: is a type of intracellular pH elevation [GO:0051454]; is part of phagosome maturation [GO:0090382] References: PMID:22008230 Sources: GOC:rjd Also known as: phagosomal reneutralization, phagosome pH elevation